ornithine racemase activity [GO:0050157] (molecular function) Definition: Catalysis of the reaction: L-ornithine = D-ornithine. Relationships: is a type of amino-acid racemase activity [GO:0047661] Sources: EC:5.1.1.12